platelet activating factor metabolic process [GO:0046469] (biological process) Definition: The chemical reactions and pathways involving platelet activating factor, 1-O-alkyl-2-acetyl-sn-glycerol 3-phosphocholine, where alkyl = hexadecyl or octadecyl. Platelet activating factor is an inflammatory mediator released from a variety of cells in response to various stimuli. Sources: ISBN:0198547684 Also known as: PAF metabolic process, PAF metabolism, platelet activating factor metabolism Relationships: is_a glycerophospholipid metabolic process [GO:0006650]; is a type of GO:0046485 Subtypes: platelet activating factor biosynthetic process [GO:0006663], platelet activating factor catabolic process [GO:0062234]